{
  "term_label": "Unknown biological process",
  "gene_symbol": "SERTAD4",
  "term_id": "UNKNOWN:0002",
  "gene": "UniProtKB:Q9NUC0",
  "gene_name": "SERTA domain-containing protein 4"
}